antimonite secondary active transmembrane transporter activity [GO:0042960] (molecular function) Definition: Enables the transfer of antimonite from one side of a membrane to the other, up its concentration gradient. The transporter binds the solute and undergoes a series of conformational changes. Transport works equally well in either direction and is driven by a chemiosmotic source of energy. Secondary active transporters include symporters and antiporters. Sources: GOC:jl Relationships: is_a GO:0015104; is a type of secondary active transmembrane transporter activity [GO:0015291] Also known as: antimonite porter activity